{
  "gene_name": "Protein MEMO1",
  "gene": "UniProtKB:Q9Y316",
  "gene_symbol": "MEMO1",
  "term_label": "Unknown biological process",
  "term_id": "UNKNOWN:0002"
}